{
  "gene": "UniProtKB:Q9HCP0",
  "gene_name": "Casein kinase I isoform gamma-1",
  "term_label": "cytoplasm",
  "term_id": "GO:0005737",
  "gene_symbol": "CSNK1G1"
}